D-sedoheptulose 7-phosphate isomerase activity [GO:0008968] (molecular function) Relationships: is_a GO:0016868 Also known as: phosphoheptose isomerase activity Definition: Catalysis of the reaction: D-sedoheptulose-7-phosphate = D-alpha,beta-D-heptose 7-phosphate. References: PMID:11279237, PMID:8631969 Sources: MetaCyc:RXN0-4301